{
  "term_label": "Unknown cellular component",
  "gene_name": "Proline-rich protein 25",
  "gene_symbol": "PRR25",
  "term_id": "UNKNOWN:0003",
  "gene": "UniProtKB:Q96S07"
}